{
  "term_id": "GO:0006357",
  "term_label": "regulation of transcription by RNA polymerase II",
  "gene": "UniProtKB:Q8N187",
  "gene_name": "Calcium-responsive transcription factor",
  "gene_symbol": "CARF"
}